{
  "gene_symbol": "RNF207",
  "term_id": "GO:0030544",
  "gene": "UniProtKB:Q6ZRF8",
  "gene_name": "RING finger protein 207",
  "term_label": "Hsp70 protein binding"
}